{
  "gene": "UniProtKB:O95990",
  "gene_name": "Actin-associated protein FAM107A",
  "term_label": "actin filament polymerization",
  "gene_symbol": "FAM107A",
  "term_id": "GO:0030041"
}